{
  "term_label": "regulation of transcription by RNA polymerase II",
  "gene_symbol": "CEBPD",
  "gene": "UniProtKB:P49716",
  "term_id": "GO:0006357",
  "gene_name": "CCAAT_enhancer-binding protein delta"
}